otolith development [GO:0048840] (biological process) Relationships: is a type of anatomical structure development [GO:0048856]; is part of GO:0048839 Definition: The process whose specific outcome is the progression of the otolith over time, from its formation to the mature structure. Sources: GOC:sr